FATZ binding [GO:0051373] (molecular function) Relationships: is a type of cytoskeletal protein binding [GO:0008092] Definition: Binding to a member of the FATZ family of proteins, filamin-, actinin-, and telethonin-binding proteins of the Z-disc of striated muscle. FATZ proteins are located in the Z-disc of the sarcomere and are involved in a complex network of interactions with other Z-band components. Also known as: FATZ 1 binding, FATZ 2 binding, FATZ 3 binding, calsarcin 1 binding, calsarcin 2 binding, calsarcin 3 binding, calsarcin binding, filamin-, actinin- and telethonin-binding protein of the Z-disc of striated muscle References: PMID:10984498, PMID:11699871